{
  "gene_symbol": "PCP4",
  "term_id": "GO:0005509",
  "term_label": "calcium ion binding",
  "gene": "UniProtKB:P48539",
  "gene_name": "Calmodulin regulator protein PCP4"
}